{
  "gene_name": "Purine nucleoside phosphorylase",
  "gene": "UniProtKB:P00491",
  "gene_symbol": "PNP",
  "term_label": "cytoplasm",
  "term_id": "GO:0005737"
}